{
  "gene_name": "Eppin",
  "term_id": "UNKNOWN:0001",
  "term_label": "Unknown molecular function",
  "gene": "UniProtKB:O95925",
  "gene_symbol": "EPPIN"
}